{
  "term_label": "chloride transmembrane transport",
  "gene_symbol": "SLC12A7",
  "term_id": "GO:1902476",
  "gene": "UniProtKB:Q9Y666",
  "gene_name": "Solute carrier family 12 member 7"
}